{
  "gene_name": "POU domain, class 3, transcription factor 2",
  "gene": "UniProtKB:P20265",
  "gene_symbol": "POU3F2",
  "term_label": "regulation of transcription by RNA polymerase II",
  "term_id": "GO:0006357"
}